CTP catabolic process [GO:0006254] (biological process) Also known as: CTP breakdown, CTP catabolism, CTP degradation, CTP hydrolysis Definition: The chemical reactions and pathways resulting in the breakdown of CTP, cytidine 5'-triphosphate. Relationships: is a type of GO:0009210; is a type of GO:0009222; is a type of CTP metabolic process [GO:0046036] Sources: ISBN:0198506732